{
  "term_label": "cytosol",
  "term_id": "GO:0005829",
  "gene": "UniProtKB:C9JLJ4",
  "gene_name": "Ubiquitin carboxyl-terminal hydrolase 17-like protein 13",
  "gene_symbol": "USP17L13"
}